somatic hypermutation of immunoglobulin genes [GO:0016446] (biological process) Also known as: somatic hypermutation of antibody genes Subtypes: somatic hypermutation of immunoglobulin genes involved in immune response [GO:0002205] Relationships: is a type of GO:0002566; is a type of somatic diversification of immunoglobulins [GO:0016445] Definition: Mutations occurring somatically that result in amino acid changes in the rearranged V regions of immunoglobulins. References: PMID:11205330, PMID:11205333, PMID:14975236, PMID:7813007 Sources: GOC:add, ISBN:0781735149